{
  "gene_name": "Vinexin",
  "term_id": "GO:0005737",
  "gene": "UniProtKB:O60504",
  "gene_symbol": "SORBS3",
  "term_label": "cytoplasm"
}